learned vocalization behavior or vocal learning [GO:0098598] (biological process) References: PMID:16418265, PMID:17035521 Sources: GOC:BHF, GOC:dos, GOC:rl Subtypes: vocal learning [GO:0042297], GO:0098583 Definition: Vocalisation behavior that is the result of learning, or the process by which new vocalizations are learned. Note: This grouping term is necessary because, in the absence of conditional mutations, it is not possible to use phenotypic evidence to distinguish an effect on vocal learning from an effect on learned vocalisation behavior. Relationships: is a type of GO:0007611